5alpha,9alpha,10beta-labda-8(20),13-dien-15-yl diphosphate biosynthetic process [GO:1901949] (biological process) Relationships: is a type of phospholipid biosynthetic process [GO:0008654]; is a type of diterpenoid biosynthetic process [GO:0016102] References: PMID:22027823 Sources: GOC:TermGenie Definition: The chemical reactions and pathways resulting in the formation of 5alpha,9alpha,10beta-labda-8(20),13-dien-15-yl diphosphate. Also known as: 5alpha,9alpha,10beta-labda-8(20),13-dien-15-yl diphosphate anabolism, 5alpha,9alpha,10beta-labda-8(20),13-dien-15-yl diphosphate biosynthesis, 5alpha,9alpha,10beta-labda-8(20),13-dien-15-yl diphosphate formation, 5alpha,9alpha,10beta-labda-8(20),13-dien-15-yl diphosphate synthesis